{
  "term_label": "Unknown molecular function",
  "gene_name": "T cell receptor alpha joining 31",
  "gene_symbol": "TRAJ31",
  "gene": "UniProtKB:A0A075B700",
  "term_id": "UNKNOWN:0001"
}